{
  "gene_name": "tRNA pseudouridine(38_39) synthase",
  "term_label": "mRNA pseudouridine synthesis",
  "gene_symbol": "PUS3",
  "term_id": "GO:1990481",
  "gene": "UniProtKB:Q9BZE2"
}